{
  "gene": "UniProtKB:Q7Z4T8",
  "term_label": "Unknown molecular function",
  "gene_name": "Inactive polypeptide N-acetylgalactosaminyltransferase-like protein 5",
  "gene_symbol": "GALNTL5",
  "term_id": "UNKNOWN:0001"
}